{
  "gene_symbol": "FASTK",
  "term_label": "ribonucleoprotein granule",
  "term_id": "GO:0035770",
  "gene": "UniProtKB:Q14296",
  "gene_name": "Fas-activated serine_threonine kinase"
}